{
  "gene_name": "E3 ubiquitin-protein ligase E3D",
  "term_label": "cytosol",
  "gene": "UniProtKB:Q7Z6J8",
  "term_id": "GO:0005829",
  "gene_symbol": "UBE3D"
}